{
  "gene_name": "Dimethylaniline monooxygenase [N-oxide-forming] 4",
  "gene_symbol": "FMO4",
  "term_label": "N,N-dimethylaniline monooxygenase activity",
  "term_id": "GO:0004499",
  "gene": "UniProtKB:P31512"
}